{
  "gene": "UniProtKB:P30041",
  "term_id": "GO:0004601",
  "gene_name": "Peroxiredoxin-6",
  "gene_symbol": "PRDX6",
  "term_label": "peroxidase activity"
}